{
  "gene": "UniProtKB:O00755",
  "gene_name": "Protein Wnt-7a",
  "term_id": "GO:0005615",
  "term_label": "extracellular space",
  "gene_symbol": "WNT7A"
}